{
  "gene_name": "Transmembrane protease serine 6",
  "gene_symbol": "TMPRSS6",
  "term_id": "GO:0008236",
  "gene": "UniProtKB:Q8IU80",
  "term_label": "serine-type peptidase activity"
}